{
  "term_label": "nucleus",
  "gene": "UniProtKB:Q9H4Q3",
  "gene_name": "PR domain zinc finger protein 13",
  "term_id": "GO:0005634",
  "gene_symbol": "PRDM13"
}